{
  "term_label": "Unknown biological process",
  "term_id": "UNKNOWN:0002",
  "gene_symbol": "PAFAH2",
  "gene_name": "Platelet-activating factor acetylhydrolase 2, cytoplasmic",
  "gene": "UniProtKB:Q99487"
}